{
  "term_id": "GO:0030199",
  "gene_name": "Collagen alpha-1(II) chain",
  "gene_symbol": "COL2A1",
  "gene": "UniProtKB:P02458",
  "term_label": "collagen fibril organization"
}